{
  "gene_symbol": "PRR27",
  "gene_name": "Proline-rich protein 27",
  "term_label": "Unknown biological process",
  "gene": "UniProtKB:Q6MZM9",
  "term_id": "UNKNOWN:0002"
}